{
  "gene_name": "Equilibrative nucleobase transporter 1",
  "gene_symbol": "SLC43A3",
  "gene": "UniProtKB:Q8NBI5",
  "term_id": "UNKNOWN:0001",
  "term_label": "Unknown molecular function"
}